{
  "gene_symbol": "AGPAT1",
  "gene_name": "1-acyl-sn-glycerol-3-phosphate acyltransferase alpha",
  "term_label": "1-acylglycerol-3-phosphate O-acyltransferase activity",
  "gene": "UniProtKB:Q99943",
  "term_id": "GO:0003841"
}